{
  "gene_name": "Homeobox protein Hox-B9",
  "gene_symbol": "HOXB9",
  "gene": "UniProtKB:P17482",
  "term_label": "anterior/posterior pattern specification",
  "term_id": "GO:0009952"
}